{
  "gene_symbol": "ALG6",
  "term_label": "dolichyl pyrophosphate Man9GlcNAc2 alpha-1,3-glucosyltransferase activity",
  "term_id": "GO:0042281",
  "gene": "UniProtKB:Q9Y672",
  "gene_name": "Dolichyl pyrophosphate Man9GlcNAc2 alpha-1,3-glucosyltransferase"
}